{
  "term_label": "Unknown molecular function",
  "gene_name": "Steroid transmembrane transporter SLC22A24",
  "gene": "UniProtKB:Q8N4F4",
  "gene_symbol": "SLC22A24",
  "term_id": "UNKNOWN:0001"
}